{
  "gene_name": "Small nuclear ribonucleoprotein-associated protein N",
  "term_id": "GO:0005687",
  "gene": "UniProtKB:P63162",
  "gene_symbol": "SNRPN",
  "term_label": "U4 snRNP"
}